smooth muscle contractile fiber [GO:0030485] (CC) Definition: The contractile fiber of smooth muscle cells. Relationships: is a type of contractile muscle fiber [GO:0043292] Sources: GOC:mah